neurofibrillary tangle assembly [GO:1902988] (biological process) Relationships: is_a inclusion body assembly [GO:0070841] References: PMID:15897157, PMID:22986780, PMID:24154541 Sources: GOC:TermGenie, GOC:sjp, GO_REF:0000079 Also known as: neurofibrillary tangle formation, flame-shaped neurofibrillary tangle assembly, flame-shaped neurofibrillary tangle formation, star-shaped neurofibrillary tangle assembly, star-shaped neurofibrillary tangle formation Note: Neurofibrillary tangles have been found in aging population; their formation is increased in Alzheimer's disease patients (and in other neurological diseases) compared to normal controls (see PMID:848276 and PMID:8584267). Definition: The aggregation, arrangement and bonding together of a set of components to form a neurofibrillary tangle. Regulation: regulated by regulation of neurofibrillary tangle assembly [GO:1902996]; negatively regulated by negative regulation of neurofibrillary tangle assembly [GO:1902997]; positively regulated by positive regulation of neurofibrillary tangle assembly [GO:1902998]